pupal development [GO:0035209] (biological process) Definition: The process whose specific outcome is the progression of the pupa over time, from its formation to the mature structure. The pupa is a dormant life stage interposed between the larval and the adult stages in insects that undergo a complete metamorphosis. Relationships: is a type of instar larval or pupal development [GO:0002165]; BFO_0000051 GO:0007562; has part apolysis [GO:0018989] Sources: GOC:bf, GOC:mtg_sensu